{
  "term_id": "GO:0006362",
  "term_label": "transcription elongation by RNA polymerase I",
  "gene": "UniProtKB:P19388",
  "gene_symbol": "POLR2E",
  "gene_name": "DNA-directed RNA polymerases I, II, and III subunit RPABC1"
}